{
  "gene": "UniProtKB:Q6NVV3",
  "gene_symbol": "NIPAL1",
  "term_id": "UNKNOWN:0001",
  "gene_name": "Magnesium transporter NIPA3",
  "term_label": "Unknown molecular function"
}